{
  "term_id": "GO:0048013",
  "gene_symbol": "EPHB3",
  "gene_name": "Ephrin type-B receptor 3",
  "term_label": "ephrin receptor signaling pathway",
  "gene": "UniProtKB:P54753"
}